{
  "gene_symbol": "TMEM128",
  "term_id": "UNKNOWN:0003",
  "gene_name": "Transmembrane protein 128",
  "term_label": "Unknown cellular component",
  "gene": "UniProtKB:Q5BJH2"
}